protein localization to ERGIC [GO:0106272] (biological process) Definition: A process in which a protein is transported to, or maintained in, a location within the endoplasmic reticulum-Golgi intermediate compartment (ERGIC). Relationships: is a type of GO:0034067 References: PMID:32272059